apolysis [GO:0018989] (biological process) Definition: The first process of molting, characterized by the detachment of the old cuticle from the underlying epidermal cells. Sources: GOC:jl Relationships: is a type of GO:0022404; is part of molting cycle, chitin-based cuticle [GO:0007591]